sarcoplasmic reticulum lumen [GO:0033018] (cellular component) Relationships: is a type of endoplasmic reticulum lumen [GO:0005788]; is part of sarcoplasmic reticulum [GO:0016529] Sources: GOC:rph Definition: The volume enclosed by the membranes of the sarcoplasmic reticulum. Subtypes: longitudinal sarcoplasmic reticulum lumen [GO:0014803], terminal cisterna lumen [GO:0014804]